{
  "term_label": "melanin biosynthetic process from tyrosine",
  "gene_symbol": "DCT",
  "gene": "UniProtKB:P40126",
  "gene_name": "L-dopachrome tautomerase",
  "term_id": "GO:0006583"
}